{
  "term_label": "epithelial structure maintenance",
  "gene": "UniProtKB:P0C091",
  "gene_name": "FRAS1-related extracellular matrix protein 3",
  "term_id": "GO:0010669",
  "gene_symbol": "FREM3"
}